{
  "gene_symbol": "CEACAM1",
  "term_label": "signal transduction",
  "gene_name": "Carcinoembryonic antigen-related cell adhesion molecule 1",
  "gene": "UniProtKB:P13688",
  "term_id": "GO:0007165"
}